{
  "term_label": "nucleus",
  "gene": "UniProtKB:Q13686",
  "gene_name": "Nucleic acid dioxygenase ALKBH1",
  "gene_symbol": "ALKBH1",
  "term_id": "GO:0005634"
}